{
  "gene": "UniProtKB:Q8NGD2",
  "term_id": "GO:0004984",
  "term_label": "olfactory receptor activity",
  "gene_name": "Olfactory receptor 4K2",
  "gene_symbol": "OR4K2"
}